dethiobiotin transmembrane transporter activity [GO:1901604] (MF) Definition: Enables the transfer of dethiobiotin from one side of a membrane to the other. Sources: GOC:TermGenie Relationships: is a type of monocarboxylic acid transmembrane transporter activity [GO:0008028]; is a type of amide transmembrane transporter activity [GO:0042887]